{
  "gene": "UniProtKB:Q92886",
  "gene_symbol": "NEUROG1",
  "term_id": "GO:0005634",
  "term_label": "nucleus",
  "gene_name": "Neurogenin-1"
}